{
  "gene_name": "Leucine-rich repeat and immunoglobulin-like domain-containing nogo receptor-interacting protein 2",
  "gene_symbol": "LINGO2",
  "term_label": "Unknown biological process",
  "gene": "UniProtKB:Q7L985",
  "term_id": "UNKNOWN:0002"
}